HLA-A specific inhibitory MHC class I receptor activity [GO:0030107] (molecular function) References: PMID:11929129, PMID:9368779 Sources: GOC:add, GOC:mah Relationships: is a type of inhibitory MHC class I receptor activity [GO:0032396] Definition: Combining with a MHC class I molecule of the HLA-A subclass to mediate signaling that inhibits activation of a lymphocyte.